p-hydroxyphenyl lignin biosynthetic process [GO:1901060] (biological process) Definition: The chemical reactions and pathways resulting in the formation of p-hydroxyphenyl lignin. Also known as: H-lignin biosynthetic process, p-hydroxyphenyl lignin anabolism, p-hydroxyphenyl lignin biosynthesis, p-hydroxyphenyl lignin formation, p-hydroxyphenyl lignin synthesis Relationships: is a type of lignin biosynthetic process [GO:0009809] Sources: GOC:TermGenie, GOC:mengo_curators